{
  "term_id": "UNKNOWN:0003",
  "gene_symbol": "CSMD2",
  "term_label": "Unknown cellular component",
  "gene_name": "CUB and sushi domain-containing protein 2",
  "gene": "UniProtKB:Q7Z408"
}